MHC protein complex [GO:0042611] (cellular component) Definition: A transmembrane protein complex composed of an MHC alpha chain and, in most cases, either an MHC class II beta chain or an invariant beta2-microglobin chain, and with or without a bound peptide, lipid, or polysaccharide antigen. References: PMID:15928678, PMID:16153240 Sources: GOC:add, GOC:jl, ISBN:0781735149 Relationships: is_a plasma membrane protein complex [GO:0098797] Subtypes: MHC class Ib protein complex [GO:0032398], MHC class I protein complex [GO:0042612], GO:0042613